{
  "gene_symbol": "SSX2IP",
  "gene_name": "Afadin- and alpha-actinin-binding protein",
  "term_label": "centriolar satellite",
  "term_id": "GO:0034451",
  "gene": "UniProtKB:Q9Y2D8"
}